{
  "gene_name": "G protein-coupled receptor kinase 5",
  "term_label": "protein kinase activity",
  "term_id": "GO:0004672",
  "gene_symbol": "GRK5",
  "gene": "UniProtKB:P34947"
}